{
  "gene_name": "Zinc finger protein 354C",
  "term_label": "RNA polymerase II cis-regulatory region sequence-specific DNA binding",
  "gene": "UniProtKB:Q86Y25",
  "gene_symbol": "ZNF354C",
  "term_id": "GO:0000978"
}